{
  "gene": "UniProtKB:Q9BXJ7",
  "term_id": "GO:0043235",
  "gene_symbol": "AMN",
  "term_label": "receptor complex",
  "gene_name": "Protein amnionless"
}